aerobic respiration, using hydrogen as electron donor [GO:0019412] (biological process) Relationships: is a type of aerobic respiration [GO:0009060]; is_a energy derivation by oxidation of reduced inorganic compounds [GO:0015975] Sources: MetaCyc:P283-PWY Definition: The oxidation of hydrogen (H2) to water (H2O), using oxygen (O2) as the electron acceptor. A hydrogenase enzyme binds H2 and the hydrogen atoms are passed through an electron transfer chain to O2 to form water. Also known as: hydrogen oxidation